vascular cord development [GO:0072360] (biological process) Definition: The progression of the vascular cord over time from its initial formation until its mature state. The vascular cord is the primordial vasculature that will develop into blood vessels by the process of tubulogenesis. References: PMID:7084422 Sources: GOC:mah, ZFA:0005077 Relationships: is a type of GO:0048856; BFO_0000050 circulatory system development [GO:0072359]